malyl-CoA lyase activity [GO:0050083] (molecular function) Sources: EC:4.1.3.24, MetaCyc:MALYL-COA-LYASE-RXN Also known as: (3S)-3-carboxy-3-hydroxypropanoyl-CoA glyoxylate-lyase (acetyl-CoA-forming), (3S)-3-carboxy-3-hydroxypropanoyl-CoA glyoxylate-lyase activity, malyl-coenzyme A lyase activity Relationships: is a type of GO:0016833 Definition: Catalysis of the reaction: (3S)-3-carboxy-3-hydroxypropanoyl-CoA = acetyl-CoA + glyoxylate.